histone H2AK15ub reader activity [GO:0140120] (MF) Note: Note that the residue position corresponds to the canonical human H2A2A histone (UniProtKB:Q6FI13); this residue is conserved across all eukaryotes. Residue 1 is the first residue following removal of the initiating Methionine (Met). Note that each histone is encoded by multiple genes, and sequences may vary across different genes within an organism. Relationships: is a type of histone H2A reader activity [GO:0140054] Definition: A histone reader that recognizes a histone H2A ubiquitinated at lysine 15. References: PMID:23760478